{
  "gene": "UniProtKB:Q8IYD1",
  "gene_symbol": "GSPT2",
  "term_id": "GO:0003924",
  "term_label": "GTPase activity",
  "gene_name": "Eukaryotic peptide chain release factor GTP-binding subunit ERF3B"
}